{
  "term_label": "galanin receptor activity",
  "term_id": "GO:0004966",
  "gene_symbol": "RXFP4",
  "gene_name": "Relaxin-3 receptor 2",
  "gene": "UniProtKB:Q8TDU9"
}